{
  "gene": "UniProtKB:Q92805",
  "term_id": "GO:0005794",
  "gene_name": "Golgin subfamily A member 1",
  "term_label": "Golgi apparatus",
  "gene_symbol": "GOLGA1"
}